GDP-fucose transmembrane transport [GO:0015783] (biological process) Also known as: GDP-fucose transport Sources: GOC:ai Subtypes: GDP-fucose import into endoplasmic reticulum lumen [GO:0036084], GO:0036085 Definition: The directed movement of GDP-fucose into, out of or within a cell, or between cells, by means of some agent such as a transporter or pore. GDP-fucose is a substance composed of fucose in glycosidic linkage with guanosine diphosphate. Relationships: is a type of purine nucleotide-sugar transmembrane transport [GO:0090480]